{
  "gene_name": "Regulator of microtubule dynamics protein 2",
  "gene": "UniProtKB:Q96LZ7",
  "term_label": "spindle microtubule",
  "term_id": "GO:0005876",
  "gene_symbol": "RMDN2"
}